{
  "term_id": "GO:0006809",
  "gene_name": "Nitric oxide synthase, inducible",
  "term_label": "nitric oxide biosynthetic process",
  "gene": "UniProtKB:P35228",
  "gene_symbol": "NOS2"
}